{
  "term_label": "plasma membrane",
  "term_id": "GO:0005886",
  "gene_name": "Coiled-coil domain-containing protein 141",
  "gene_symbol": "CCDC141",
  "gene": "UniProtKB:Q6ZP82"
}